{
  "gene_name": "Dynein regulatory complex subunit 2",
  "gene": "UniProtKB:Q8IXS2",
  "gene_symbol": "CCDC65",
  "term_id": "UNKNOWN:0001",
  "term_label": "Unknown molecular function"
}